long-chain fatty acid import across plasma membrane [GO:0015911] (biological process) Note: While there is not universal consensus on the lengths of short-, medium-, long- and very-long-chain fatty acids, the GO uses the definitions in ChEBI (see CHEBI:26666, CHEBI:59554, CHEBI:15904 and CHEBI:27283). Definition: The directed movement of a long-chain fatty acid from outside of a cell, across the plasma membrane and into the cytosol. A long-chain fatty acid has an aliphatic tail containing 13 to 22 carbons. Also known as: plasma membrane long-chain fatty acid transport Sources: GOC:ai Regulation: RO_0002211 by regulation of long-chain fatty acid import across plasma membrane [GO:0010746]; positively regulated by positive regulation of long-chain fatty acid import across plasma membrane [GO:0010747]; negatively regulated by GO:0010748 Relationships: is a type of long-chain fatty acid import into cell [GO:0044539]; is a type of GO:0098739; is_a fatty acid transmembrane transport [GO:1902001]